transmembrane receptor protein kinase activity [GO:0019199] (molecular function) Definition: Combining with a signal and transmitting the signal from one side of the membrane to the other to initiate a change in cell activity by catalysis of the reaction: a protein + ATP = a phosphoprotein + ADP. Subtypes: transmembrane receptor protein serine/threonine kinase activity [GO:0004675], transmembrane receptor protein tyrosine kinase activity [GO:0004714], GO:0009784 Sources: GOC:mah Relationships: is a type of protein kinase activity [GO:0004672]; is a type of GO:0004888